{
  "gene": "UniProtKB:Q9Y5S8",
  "term_label": "superoxide anion generation",
  "gene_name": "NADPH oxidase 1",
  "gene_symbol": "NOX1",
  "term_id": "GO:0042554"
}